{
  "gene": "UniProtKB:P08319",
  "term_label": "zinc ion binding",
  "gene_symbol": "ADH4",
  "gene_name": "All-trans-retinol dehydrogenase [NAD(+)] ADH4",
  "term_id": "GO:0008270"
}